organellar chromatophore outer membrane [GO:0070114] (cellular component) Relationships: is a type of peribacteroid membrane [GO:0043661]; is a type of GO:0070112 Sources: GOC:mah Also known as: Paulinella-type chromatophore outer membrane Definition: The outer, i.e. cytoplasm-facing, of the two lipid bilayers surrounding an organellar chromatophore.